{
  "gene": "UniProtKB:O00629",
  "term_id": "GO:0042564",
  "gene_name": "Importin subunit alpha-3",
  "term_label": "NLS-dependent protein nuclear import complex",
  "gene_symbol": "KPNA4"
}